90S preribosome assembly [GO:0034463] (BP) Sources: GOC:krc, GOC:mah, GOC:tb Definition: The aggregation, arrangement and bonding together of proteins and RNA molecules to form a 90S preribosome. The 90S preribosome represents the complex that forms on the primary rRNA transcript before it splits into the small subunit and large subunit portions. Relationships: is a type of protein-RNA complex assembly [GO:0022618]; is part of cytosolic ribosome assembly [GO:0042256]